{
  "term_id": "UNKNOWN:0001",
  "gene": "UniProtKB:Q9P086",
  "gene_symbol": "MED11",
  "term_label": "Unknown molecular function",
  "gene_name": "Mediator of RNA polymerase II transcription subunit 11"
}